{
  "gene": "UniProtKB:Q9BXL7",
  "term_id": "GO:0035591",
  "gene_name": "Caspase recruitment domain-containing protein 11",
  "term_label": "signaling adaptor activity",
  "gene_symbol": "CARD11"
}